{
  "gene": "UniProtKB:A0A3B3IU46",
  "gene_name": "RNA guanine-N7 methyltransferase-activating subunit-like protein",
  "gene_symbol": "RAMACL",
  "term_label": "7-methylguanosine mRNA capping",
  "term_id": "GO:0006370"
}